{
  "gene_name": "Zinc finger CCCH domain-containing protein 10",
  "term_id": "GO:0003723",
  "term_label": "RNA binding",
  "gene_symbol": "ZC3H10",
  "gene": "UniProtKB:Q96K80"
}